membrane grommet activity [GO:0180024] (molecular function) Relationships: is a type of molecular_function [GO:0003674] Definition: An activity in which a protein, or group of proteins, acts to restrict the size of a fenestration in a membrane or membrane system (i.e. restrict the diameter of a hole in a membrane). An example of this is the molecular function is performed by ESCRT-III proteins at the nuclear envelope of fission yeast during anaphase B. References: PMID:37783794